positive regulation of B cell activation [GO:0050871] (biological process) Subtypes: GO:0030890, B cell costimulation [GO:0031296], positive regulation of B cell differentiation [GO:0045579], GO:0045830 Relationships: is_a regulation of B cell activation [GO:0050864]; is a type of positive regulation of lymphocyte activation [GO:0051251]; positively regulates B cell activation [GO:0042113] Sources: GOC:ai Definition: Any process that activates or increases the frequency, rate or extent of B cell activation. Also known as: positive regulation of B lymphocyte activation, positive regulation of B-cell activation, positive regulation of B-lymphocyte activation, up regulation of B cell activation, up-regulation of B cell activation, upregulation of B cell activation, activation of B cell activation, stimulation of B cell activation